{
  "gene_name": "Serine--tRNA ligase, cytoplasmic",
  "term_id": "GO:0006434",
  "term_label": "seryl-tRNA aminoacylation",
  "gene_symbol": "SARS1",
  "gene": "UniProtKB:P49591"
}